{
  "gene_name": "E3 ubiquitin-protein ligase TRIM71",
  "gene_symbol": "TRIM71",
  "gene": "UniProtKB:Q2Q1W2",
  "term_id": "GO:0000209",
  "term_label": "protein polyubiquitination"
}